{
  "gene_name": "Cilia- and flagella-associated protein 70",
  "gene": "UniProtKB:Q5T0N1",
  "term_id": "GO:0060271",
  "term_label": "cilium assembly",
  "gene_symbol": "CFAP70"
}